{
  "term_id": "GO:0051123",
  "gene_symbol": "TAF7",
  "term_label": "RNA polymerase II preinitiation complex assembly",
  "gene": "UniProtKB:Q15545",
  "gene_name": "Transcription initiation factor TFIID subunit 7"
}